PTW/PP1 phosphatase complex [GO:0072357] (cellular component) Relationships: is a type of protein phosphatase type 1 complex [GO:0000164] References: PMID:20516061 Sources: GOC:mah Definition: A protein serine/threonine phosphatase complex that contains a catalytic subunit (PPP1CA, PPP1CB or PPP1CC) and the regulatory subunits PPP1R10 (PNUTS), TOX4 and WDR82, and plays a role in the control of chromatin structure and cell cycle progression during the transition from mitosis into interphase.